positive regulation of type II interferon production [GO:0032729] (biological process) Relationships: is a type of positive regulation of cytokine production [GO:0001819]; is a type of regulation of type II interferon production [GO:0032649]; positively regulates type II interferon production [GO:0032609] Also known as: positive regulation of interferon-gamma production, up regulation of interferon-gamma production, up-regulation of interferon-gamma production, upregulation of interferon-gamma production, activation of interferon-gamma production, positive regulation of interferon-gamma biosynthetic process, positive regulation of interferon-gamma secretion, stimulation of interferon-gamma production References: PMID:15546383 Sources: GOC:add, GOC:mah Definition: Any process that activates or increases the frequency, rate, or extent of interferon-gamma production. Interferon-gamma is also known as type II interferon.